{
  "term_id": "GO:0050892",
  "gene_name": "Junctional adhesion molecule A",
  "term_label": "intestinal absorption",
  "gene_symbol": "F11R",
  "gene": "UniProtKB:Q9Y624"
}